phosphorylase kinase complex [GO:0005964] (cellular component) Definition: An enzyme complex that catalyzes the phosphorylation of phosphorylase b to form phosphorylase a. Relationships: is a type of GO:1902554; is part of cytoplasm [GO:0005737] References: PMID:1370475